chorio-allantoic fusion [GO:0060710] (biological process) Sources: GOC:dph Definition: The cell-cell adhesion process in which the cells of the chorion fuse to the cells of the allantois. Relationships: is a type of cell-cell adhesion [GO:0098609]; is part of labyrinthine layer morphogenesis [GO:0060713]